regulation of ERBB3 signaling pathway [GO:1905578] (biological process) References: PMID:27353365 Sources: GOC:TermGenie, GOC:als, GO_REF:0000058 Subtypes: negative regulation of ERBB3 signaling pathway [GO:1905579], positive regulation of ERBB3 signaling pathway [GO:1905580] Relationships: is a type of regulation of ERBB signaling pathway [GO:1901184]; regulates ERBB3 signaling pathway [GO:0038129] Definition: Any process that modulates the frequency, rate or extent of ERBB3 signaling pathway. Also known as: regulation of ERBB3 signalling pathway, regulation of HER3 signaling pathway, regulation of receptor tyrosine-protein kinase erbB-3 signaling pathway